{
  "term_id": "GO:0005634",
  "term_label": "nucleus",
  "gene_name": "PAK4-inhibitor INKA1",
  "gene_symbol": "INKA1",
  "gene": "UniProtKB:Q96EL1"
}